negative regulation of nodal signaling pathway [GO:1900108] (biological process) Sources: GOC:BHF, GOC:TermGenie, GOC:vk Definition: Any process that stops, prevents or reduces the frequency, rate or extent of nodal signaling pathway. Also known as: down regulation of nodal signaling, down regulation of nodal signaling pathway, down-regulation of nodal signaling, down-regulation of nodal signaling pathway, downregulation of nodal signaling, downregulation of nodal signaling pathway, negative regulation of nodal signaling, negative regulation of nodal signalling pathway, inhibition of nodal signaling, inhibition of nodal signaling pathway Relationships: is a type of negative regulation of activin receptor signaling pathway [GO:0032926]; is a type of regulation of nodal signaling pathway [GO:1900107]; negatively regulates nodal signaling pathway [GO:0038092]